{
  "gene_name": "Leucine-rich repeat and immunoglobulin-like domain-containing nogo receptor-interacting protein 3",
  "term_id": "UNKNOWN:0002",
  "term_label": "Unknown biological process",
  "gene_symbol": "LINGO3",
  "gene": "UniProtKB:P0C6S8"
}